{
  "gene_name": "Elongation factor 2",
  "gene": "UniProtKB:P13639",
  "term_label": "ribosome binding",
  "term_id": "GO:0043022",
  "gene_symbol": "EEF2"
}